{
  "term_id": "GO:0005886",
  "term_label": "plasma membrane",
  "gene_name": "Leucine-rich repeat neuronal protein 3",
  "gene": "UniProtKB:Q9H3W5",
  "gene_symbol": "LRRN3"
}